{
  "term_label": "nucleus",
  "gene": "UniProtKB:P02511",
  "gene_name": "Alpha-crystallin B chain",
  "term_id": "GO:0005634",
  "gene_symbol": "CRYAB"
}